{
  "gene_symbol": "SGTA",
  "gene": "UniProtKB:O43765",
  "term_id": "GO:0016020",
  "term_label": "membrane",
  "gene_name": "Small glutamine-rich tetratricopeptide repeat-containing protein alpha"
}